{
  "term_id": "GO:0160125",
  "gene": "UniProtKB:Q9UHC3",
  "term_label": "pH-gated sodium channel activity",
  "gene_symbol": "ASIC3",
  "gene_name": "Acid-sensing ion channel 3"
}